{
  "gene_symbol": "EEF1A1",
  "term_id": "GO:0003746",
  "gene_name": "Elongation factor 1-alpha 1",
  "term_label": "translation elongation factor activity",
  "gene": "UniProtKB:P68104"
}